recycling of RNA polymerase [GO:0140182] (biological process) Definition: The process of freeing aborted or stalled RNA polymerase (RNAP), which dissociates it from nucleic acids and allows RNAP to reinitiate another transcription cycle. The freed mRNA is not used for further transcription. Relationships: is_a cellular homeostasis [GO:0019725]; is part of DNA-templated transcription termination [GO:0006353] References: PMID:33339820, PMID:33339823, PMID:33339827, PMID:39384756